regulation of transforming growth factor beta1 production [GO:0032908] (biological process) Relationships: is a type of regulation of transforming growth factor beta production [GO:0071634]; regulates transforming growth factor beta1 production [GO:0032905] Subtypes: GO:0032911, GO:0032914 Definition: Any process that modulates the frequency, rate, or extent of production of transforming growth factor-beta1. Also known as: regulation of TGF-B1 production, regulation of TGFB1 production, regulation of transforming growth factor-beta1 production Sources: GOC:mah